{
  "term_id": "UNKNOWN:0003",
  "gene_name": "EF-hand calcium-binding domain-containing protein 5",
  "gene_symbol": "EFCAB5",
  "term_label": "Unknown cellular component",
  "gene": "UniProtKB:A4FU69"
}